{
  "gene_symbol": "UGT1A7",
  "term_label": "endoplasmic reticulum",
  "gene": "UniProtKB:Q9HAW7",
  "term_id": "GO:0005783",
  "gene_name": "UDP-glucuronosyltransferase 1A7"
}